{
  "gene_name": "Probable 18S rRNA (guanine-N(7))-methyltransferase",
  "term_label": "nucleolus",
  "gene_symbol": "BUD23",
  "gene": "UniProtKB:O43709",
  "term_id": "GO:0005730"
}